{
  "gene_symbol": "P2RY6",
  "term_label": "cellular response to pyrimidine ribonucleotide",
  "term_id": "GO:1905835",
  "gene": "UniProtKB:Q15077",
  "gene_name": "P2Y purinoceptor 6"
}